{
  "gene_name": "SH3 domain-binding protein 1",
  "gene_symbol": "SH3BP1",
  "gene": "UniProtKB:Q9Y3L3",
  "term_label": "cytosol",
  "term_id": "GO:0005829"
}